{
  "gene": "UniProtKB:Q16584",
  "term_label": "microtubule-based process",
  "term_id": "GO:0007017",
  "gene_symbol": "MAP3K11",
  "gene_name": "Mitogen-activated protein kinase kinase kinase 11"
}